{
  "gene_symbol": "APCDD1L",
  "gene_name": "Protein APCDD1-like",
  "term_label": "Unknown biological process",
  "gene": "UniProtKB:Q8NCL9",
  "term_id": "UNKNOWN:0002"
}